{
  "gene": "UniProtKB:Q96JB1",
  "gene_name": "Dynein axonemal heavy chain 8",
  "gene_symbol": "DNAH8",
  "term_id": "GO:0036157",
  "term_label": "outer dynein arm"
}